IAA-Ala conjugate hydrolase activity [GO:0010179] (molecular function) Definition: Catalysis of the reaction: indole-3-acetyl-alanine + H2O = indole-3-acetate + L-alanine. Sources: MetaCyc:RXN-2981 Relationships: is a type of IAA-amino acid conjugate hydrolase activity [GO:0010178]